{
  "term_label": "regulation of transcription by RNA polymerase II",
  "term_id": "GO:0006357",
  "gene_name": "Zinc finger and BTB domain-containing protein 18",
  "gene_symbol": "ZBTB18",
  "gene": "UniProtKB:Q99592"
}